{
  "gene_name": "TATA box-binding protein-associated factor RNA polymerase I subunit D",
  "term_label": "nucleoplasm",
  "gene": "UniProtKB:Q9H5J8",
  "gene_symbol": "TAF1D",
  "term_id": "GO:0005654"
}